{
  "term_id": "GO:0032391",
  "gene_symbol": "RP1L1",
  "term_label": "photoreceptor connecting cilium",
  "gene": "UniProtKB:Q8IWN7",
  "gene_name": "Retinitis pigmentosa 1-like 1 protein"
}